{
  "gene": "UniProtKB:O15245",
  "gene_name": "Solute carrier family 22 member 1",
  "term_id": "UNKNOWN:0003",
  "term_label": "Unknown cellular component",
  "gene_symbol": "SLC22A1"
}